nuclear pore inner ring [GO:0044611] (cellular component) Definition: A subcomplex of the nuclear pore complex (NPC) that forms the inner rings of the core scaffold, a lattice-like structure that gives the NPC its shape and strength. In S. cerevisiae, the two inner rings are each composed of Nup192p, Nup188p, Nup170p and Nup157p. In vertebrates, the two inner rings are each composed of Nup205, Nup188 and Nup155. Components are arranged in 8-fold symmetrical 'spokes' around the central transport channel. A single 'spoke', can be isolated and is sometimes referred to as the Nup170 complex. References: PMID:18046406, PMID:19524430, PMID:20947011, PMID:22419078 Sources: GOC:dgf Also known as: Nup170 complex Relationships: is a type of nuclear protein-containing complex [GO:0140513]; is part of nuclear pore [GO:0005643]